collagen fibril organization [GO:0030199] (biological process) Sources: GOC:mah, ISBN:0815316194 Relationships: is a type of extracellular matrix organization [GO:0030198] Also known as: collagen fibril organisation, fibrillar collagen organization Regulation: regulated by GO:1904026; negatively regulated by negative regulation of collagen fibril organization [GO:1904027]; positively regulated by positive regulation of collagen fibril organization [GO:1904028] Definition: Any process that determines the size and arrangement of collagen fibrils within an extracellular matrix.